{
  "term_id": "UNKNOWN:0002",
  "gene_name": "Multiple epidermal growth factor-like domains protein 6",
  "gene_symbol": "MEGF6",
  "term_label": "Unknown biological process",
  "gene": "UniProtKB:O75095"
}